{
  "gene_name": "Early growth response protein 1",
  "gene": "UniProtKB:P18146",
  "gene_symbol": "EGR1",
  "term_label": "DNA-binding transcription factor activity, RNA polymerase II-specific",
  "term_id": "GO:0000981"
}